{
  "term_label": "nucleus",
  "gene_name": "Meiosis expressed gene 1 protein homolog",
  "gene": "UniProtKB:Q5JSS6",
  "gene_symbol": "MEIG1",
  "term_id": "GO:0005634"
}